{
  "gene": "UniProtKB:P16885",
  "term_label": "positive regulation of epithelial cell migration",
  "term_id": "GO:0010634",
  "gene_symbol": "PLCG2",
  "gene_name": "1-phosphatidylinositol 4,5-bisphosphate phosphodiesterase gamma-2"
}